{
  "gene": "UniProtKB:O75157",
  "term_id": "UNKNOWN:0003",
  "gene_name": "TSC22 domain family protein 2",
  "gene_symbol": "TSC22D2",
  "term_label": "Unknown cellular component"
}